bacteriocin transport [GO:0043213] (biological process) Definition: The directed movement of a bacteriocin into, out of or within a cell, or between cells, by means of some agent such as a transporter or pore. Bacteriocins are a group of antibiotics produced by bacteria and are encoded by a group of naturally occurring plasmids, e.g. Col E1. Bacteriocins are toxic to bacteria closely related to the bacteriocin producing strain. Sources: GOC:mlg Relationships: is_a amide transport [GO:0042886] Subtypes: GO:0042914